{
  "term_label": "regulation of transcription by RNA polymerase II",
  "term_id": "GO:0006357",
  "gene_symbol": "NUPR2",
  "gene": "UniProtKB:A6NF83",
  "gene_name": "Nuclear protein 2"
}